{
  "gene_symbol": "ERCC3",
  "gene": "UniProtKB:P19447",
  "term_id": "GO:0006367",
  "term_label": "transcription initiation at RNA polymerase II promoter",
  "gene_name": "General transcription and DNA repair factor IIH helicase subunit XPB"
}